{
  "gene": "UniProtKB:O60566",
  "term_label": "meiotic sister chromatid cohesion, centromeric",
  "term_id": "GO:0051754",
  "gene_symbol": "BUB1B",
  "gene_name": "Mitotic checkpoint serine_threonine-protein kinase BUB1 beta"
}